substance K receptor activity [GO:0016497] (molecular function) Relationships: is a type of tachykinin receptor activity [GO:0004995] Definition: Combining with substance K, the peptide His-Lys-Thr-Asp-Ser-Phe-Val-Gly-Leu-Met, to initiate a change in cell activity. Sources: GOC:mah, ISBN:0198506732 Also known as: neurokinin A receptor activity, neuromedin L receptor activity